{
  "gene_name": "Transcriptional enhancer factor TEF-3",
  "gene": "UniProtKB:Q15561",
  "term_label": "regulation of transcription by RNA polymerase II",
  "term_id": "GO:0006357",
  "gene_symbol": "TEAD4"
}